positive regulation of immunoglobulin production [GO:0002639] (biological process) Subtypes: positive regulation of isotype switching [GO:0045830], positive regulation of immunoglobulin production in mucosal tissue [GO:2000558] Definition: Any process that activates or increases the frequency, rate, or extent of immunoglobulin production. Relationships: is a type of regulation of immunoglobulin production [GO:0002637]; is a type of GO:0002702; positively regulates immunoglobulin production [GO:0002377] Also known as: up regulation of immunoglobulin production, up-regulation of immunoglobulin production, upregulation of immunoglobulin production, activation of immunoglobulin production, positive regulation of immunoglobulin biosynthetic process, positive regulation of immunoglobulin secretion, stimulation of immunoglobulin production Sources: GOC:add